{
  "term_id": "UNKNOWN:0003",
  "gene_symbol": "KRTAP21-1",
  "gene": "UniProtKB:Q3LI58",
  "gene_name": "Keratin-associated protein 21-1",
  "term_label": "Unknown cellular component"
}